{
  "gene_symbol": "BRF1",
  "gene": "UniProtKB:Q92994",
  "term_id": "GO:0000126",
  "term_label": "transcription factor TFIIIB complex",
  "gene_name": "Transcription factor IIIB 90 kDa subunit"
}